negative regulation of protein localization to phagocytic vesicle [GO:1905170] (biological process) Definition: Any process that stops, prevents or reduces the frequency, rate or extent of protein localization to phagocytic vesicle. Also known as: down regulation of protein localisation in phagocytic vesicle, down regulation of protein localisation to phagocytic vesicle, down regulation of protein localisation to phagosome, down regulation of protein localization in phagocytic vesicle, down regulation of protein localization to phagocytic vesicle, down regulation of protein recruitment to phagosome, down-regulation of protein localisation in phagocytic vesicle, down-regulation of protein localisation to phagocytic vesicle, down-regulation of protein localisation to phagosome, down-regulation of protein localization in phagocytic vesicle, down-regulation of protein localization to phagocytic vesicle, down-regulation of protein recruitment to phagosome, downregulation of protein localisation in phagocytic vesicle, downregulation of protein localisation to phagocytic vesicle, downregulation of protein localisation to phagosome, downregulation of protein localization in phagocytic vesicle, downregulation of protein localization to phagocytic vesicle, downregulation of protein recruitment to phagosome, negative regulation of protein localisation in phagocytic vesicle, negative regulation of protein localisation to phagocytic vesicle, negative regulation of protein localisation to phagosome, negative regulation of protein localization in phagocytic vesicle, negative regulation of protein recruitment to phagosome, inhibition of protein localisation in phagocytic vesicle, inhibition of protein localisation to phagocytic vesicle, inhibition of protein localisation to phagosome, inhibition of protein localization in phagocytic vesicle, inhibition of protein localization to phagocytic vesicle, inhibition of protein recruitment to phagosome Sources: GOC:PARL, GOC:TermGenie, GOC:bf, GO_REF:0000058 Relationships: is a type of negative regulation of protein localization [GO:1903828]; is a type of regulation of protein localization to phagocytic vesicle [GO:1905169]; negatively regulates protein localization to phagocytic vesicle [GO:1905161]